{
  "term_id": "UNKNOWN:0003",
  "term_label": "Unknown cellular component",
  "gene": "UniProtKB:Q86TZ1",
  "gene_symbol": "TTC6",
  "gene_name": "Tetratricopeptide repeat protein 6"
}